{
  "term_label": "Unknown molecular function",
  "gene_symbol": "USP41",
  "gene_name": "Putative ubiquitin carboxyl-terminal hydrolase 41",
  "term_id": "UNKNOWN:0001",
  "gene": "UniProtKB:Q3LFD5"
}